{
  "gene_symbol": "USP17L30",
  "gene_name": "Ubiquitin carboxyl-terminal hydrolase 17-like protein 24",
  "term_label": "cytosol",
  "term_id": "GO:0005829",
  "gene": "UniProtKB:Q0WX57"
}